fatty acid in-chain hydroxylase activity [GO:0052722] (molecular function) Relationships: is a type of GO:0004497 Definition: Catalysis of the reaction: fatty acid + O2 + 2 NADPH + H+ = fatty acid with in-chain hydroxy group + 2 NADP+ + H2O. Sources: MetaCyc:RXN-12186